iron-sulfur cluster assembly complex [GO:1990229] (cellular component) Relationships: is a type of protein-containing complex [GO:0032991]; is part of GO:0005737 Also known as: Fe-S cluster assembly complex, SufBCD complex References: PMID:17350958 Sources: GOC:bhm Definition: A protein complex capable of assembling an iron-sulfur (Fe-S) cluster. Subtypes: cytosolic [4Fe-4S] assembly targeting complex [GO:0097361], mitochondrial [2Fe-2S] assembly complex [GO:0099128], mitochondrial [4Fe-4S] assembly complex [GO:0120510], cytosolic [4Fe-4S] assembly scaffold complex [GO:1904564], IscS-IscU complex [GO:1990330]